{
  "gene_symbol": "NINJ2",
  "gene": "UniProtKB:Q9NZG7",
  "gene_name": "Ninjurin-2",
  "term_id": "GO:0098632",
  "term_label": "cell-cell adhesion mediator activity"
}